{
  "term_id": "GO:0005739",
  "term_label": "mitochondrion",
  "gene": "UniProtKB:O43708",
  "gene_name": "Maleylacetoacetate isomerase",
  "gene_symbol": "GSTZ1"
}